{
  "term_id": "UNKNOWN:0002",
  "gene": "UniProtKB:Q9H339",
  "gene_name": "Olfactory receptor 51B5",
  "term_label": "Unknown biological process",
  "gene_symbol": "OR51B5"
}